{
  "term_id": "GO:0000028",
  "gene": "UniProtKB:P62857",
  "gene_name": "Small ribosomal subunit protein eS28",
  "gene_symbol": "RPS28",
  "term_label": "ribosomal small subunit assembly"
}